positive regulation of transcription of nucleolar large rRNA by RNA polymerase I [GO:1901838] (biological process) Relationships: is a type of positive regulation of transcription by RNA polymerase I [GO:0045943]; is_a regulation of transcription of nucleolar large rRNA by RNA polymerase I [GO:1901836]; positively regulates nucleolar large rRNA transcription by RNA polymerase I [GO:0042790] Sources: GOC:TermGenie, GOC:sart Definition: Any process that activates or increases the frequency, rate or extent of transcription of nuclear large rRNA mediated by RNA polymerase I. Also known as: activation of transcription of nuclear rRNA large Pol I transcript, positive regulation of transcription of nuclear large rRNA transcript from RNA polymerase I promoter, positive regulation of transcription of nuclear rRNA large Pol I transcript, up regulation of transcription of nuclear large rRNA transcript from RNA polymerase I promoter, up regulation of transcription of nuclear rRNA large Pol I transcript, up-regulation of transcription of nuclear large rRNA transcript from RNA polymerase I promoter, up-regulation of transcription of nuclear rRNA large Pol I transcript, upregulation of transcription of nuclear large rRNA transcript from RNA polymerase I promoter, upregulation of transcription of nuclear rRNA large Pol I transcript, activation of transcription of nuclear large rRNA transcript from RNA polymerase I promoter